{
  "gene": "UniProtKB:Q9H489",
  "gene_name": "Putative testis-specific Y-encoded-like protein 3",
  "term_id": "GO:0000785",
  "gene_symbol": "TSPY26P",
  "term_label": "chromatin"
}